pigment granule maturation [GO:0048757] (biological process) Definition: Steps required to form a membrane-bounded organelle into a pigment granule containing pigment. Maturation is a developmental process, independent of morphogenetic (shape) change, that is required for a cell or structure to attain its fully functional state. Sources: GOC:dgh, GOC:jid, GOC:mh Relationships: is a type of developmental maturation [GO:0021700]; is a type of GO:0043482; is part of pigment cell differentiation [GO:0050931]